{
  "gene_name": "WASH complex subunit 5",
  "term_label": "endosome",
  "gene": "UniProtKB:Q12768",
  "gene_symbol": "WASHC5",
  "term_id": "GO:0005768"
}